{
  "term_label": "Unknown molecular function",
  "term_id": "UNKNOWN:0001",
  "gene": "UniProtKB:Q8IWB6",
  "gene_symbol": "TEX14",
  "gene_name": "Inactive serine_threonine-protein kinase TEX14"
}